{
  "gene_name": "Protein Frey 1",
  "gene_symbol": "FREY1",
  "term_id": "GO:0005789",
  "gene": "UniProtKB:C9JXX5",
  "term_label": "endoplasmic reticulum membrane"
}